{
  "gene_symbol": "NUDCD1",
  "gene": "UniProtKB:Q96RS6",
  "gene_name": "NudC domain-containing protein 1",
  "term_label": "Unknown cellular component",
  "term_id": "UNKNOWN:0003"
}